{
  "term_id": "GO:0000398",
  "gene_symbol": "DHX8",
  "term_label": "mRNA splicing, via spliceosome",
  "gene_name": "ATP-dependent RNA helicase DHX8",
  "gene": "UniProtKB:Q14562"
}